{
  "gene": "UniProtKB:Q8IUK8",
  "gene_symbol": "CBLN2",
  "term_id": "GO:0043083",
  "term_label": "synaptic cleft",
  "gene_name": "Cerebellin-2"
}